{
  "gene_symbol": "LIME1",
  "term_label": "B cell receptor complex",
  "gene_name": "Lck-interacting transmembrane adapter 1",
  "gene": "UniProtKB:Q9H400",
  "term_id": "GO:0019815"
}